{
  "gene": "UniProtKB:Q8TE12",
  "term_label": "regulation of transcription by RNA polymerase II",
  "gene_name": "LIM homeobox transcription factor 1-alpha",
  "term_id": "GO:0006357",
  "gene_symbol": "LMX1A"
}